{
  "gene": "UniProtKB:P42702",
  "term_id": "GO:0043235",
  "term_label": "receptor complex",
  "gene_name": "Leukemia inhibitory factor receptor",
  "gene_symbol": "LIFR"
}